{
  "term_id": "UNKNOWN:0002",
  "gene_name": "Protein shisa-3 homolog",
  "term_label": "Unknown biological process",
  "gene_symbol": "SHISA3",
  "gene": "UniProtKB:A0PJX4"
}